{
  "gene_symbol": "PANO1",
  "term_label": "nucleolus",
  "term_id": "GO:0005730",
  "gene": "UniProtKB:I0J062",
  "gene_name": "Proapoptotic nucleolar protein 1"
}